{
  "gene_symbol": "SNX6",
  "term_label": "retrograde transport, endosome to Golgi",
  "term_id": "GO:0042147",
  "gene_name": "Sorting nexin-6",
  "gene": "UniProtKB:Q9UNH7"
}